{
  "term_id": "GO:0001764",
  "term_label": "neuron migration",
  "gene": "UniProtKB:O75553",
  "gene_symbol": "DAB1",
  "gene_name": "Disabled homolog 1"
}